{
  "term_id": "GO:0005737",
  "term_label": "cytoplasm",
  "gene_name": "Myosin-11",
  "gene": "UniProtKB:P35749",
  "gene_symbol": "MYH11"
}